{
  "term_label": "structural constituent of chromatin",
  "gene_symbol": "H2AC19",
  "term_id": "GO:0030527",
  "gene": "UniProtKB:Q6FI13",
  "gene_name": "Histone H2A type 2-A"
}